{
  "gene_name": "Cyclin-Y-like protein 2",
  "term_label": "plasma membrane",
  "gene": "UniProtKB:Q5T2Q4",
  "gene_symbol": "CCNYL2",
  "term_id": "GO:0005886"
}